{
  "term_id": "GO:0008076",
  "term_label": "voltage-gated potassium channel complex",
  "gene": "UniProtKB:P56696",
  "gene_symbol": "KCNQ4",
  "gene_name": "Potassium voltage-gated channel subfamily KQT member 4"
}